{
  "term_id": "UNKNOWN:0001",
  "term_label": "Unknown molecular function",
  "gene_symbol": "C5orf52",
  "gene_name": "Uncharacterized protein C5orf52",
  "gene": "UniProtKB:A6NGY3"
}